{
  "gene": "UniProtKB:P05093",
  "term_id": "GO:0042448",
  "gene_name": "Steroid 17-alpha-hydroxylase_17,20 lyase",
  "gene_symbol": "CYP17A1",
  "term_label": "progesterone metabolic process"
}